{
  "gene_name": "Uncharacterized protein C11orf86",
  "term_id": "UNKNOWN:0002",
  "term_label": "Unknown biological process",
  "gene_symbol": "C11orf86",
  "gene": "UniProtKB:A6NJI1"
}